glycine transport [GO:0015816] (biological process) Relationships: is a type of organic cation transport [GO:0015695]; is a type of GO:0015804; is a type of carboxylic acid transport [GO:0046942]; is a type of GO:0071705 Subtypes: glycine secretion [GO:0061536], glycine import across plasma membrane [GO:1903804], glycine import into mitochondrion [GO:1904983] Sources: GOC:ai Definition: The directed movement of glycine, aminoethanoic acid, into, out of or within a cell, or between cells, by means of some agent such as a transporter or pore.